{
  "term_id": "GO:0000086",
  "gene_name": "Cyclin-dependent kinase 14",
  "term_label": "G2/M transition of mitotic cell cycle",
  "gene_symbol": "CDK14",
  "gene": "UniProtKB:O94921"
}